{
  "gene": "UniProtKB:Q9UMY1",
  "term_id": "UNKNOWN:0001",
  "gene_name": "Nucleolar protein 7",
  "term_label": "Unknown molecular function",
  "gene_symbol": "NOL7"
}